{
  "gene": "UniProtKB:Q9NY12",
  "gene_symbol": "GAR1",
  "term_label": "snoRNA guided rRNA pseudouridine synthesis",
  "term_id": "GO:0000454",
  "gene_name": "H_ACA ribonucleoprotein complex subunit 1"
}